chiral amino acid racemization [GO:0018366] (biological process) Definition: The formation of a mixture of the two possible enantiomers from the D- or L-enantiomer of a chiral amino acid. Subtypes: GO:0018085 Sources: GOC:jsg, ISBN:0198506732 Relationships: is a type of GO:0006520